{
  "gene_name": "Adenylate cyclase type 3",
  "term_id": "GO:0007189",
  "gene_symbol": "ADCY3",
  "term_label": "adenylate cyclase-activating G protein-coupled receptor signaling pathway",
  "gene": "UniProtKB:O60266"
}